{
  "term_label": "mitotic cell cycle",
  "gene_symbol": "TUBG1",
  "gene_name": "Tubulin gamma-1 chain",
  "gene": "UniProtKB:P23258",
  "term_id": "GO:0000278"
}